{
  "term_id": "GO:0047676",
  "term_label": "arachidonate-CoA ligase activity",
  "gene_symbol": "ACSL4",
  "gene": "UniProtKB:O60488",
  "gene_name": "Long-chain-fatty-acid--CoA ligase 4"
}